{
  "gene_symbol": "KTN1",
  "gene": "UniProtKB:Q86UP2",
  "gene_name": "Kinectin",
  "term_label": "Unknown cellular component",
  "term_id": "UNKNOWN:0003"
}